{
  "gene": "UniProtKB:Q8IX07",
  "gene_symbol": "ZFPM1",
  "term_id": "GO:0000122",
  "gene_name": "Zinc finger protein ZFPM1",
  "term_label": "negative regulation of transcription by RNA polymerase II"
}